SLAC complex [GO:0140224] (CC) Definition: A protein complex that regulates Arp2/3 complex-mediated actin nucleation. Relationships: is a type of protein-containing complex [GO:0032991] References: PMID:22973053 Sources: GOC:lnp